{
  "term_label": "cytokine activity",
  "gene_name": "Interferon omega-1",
  "gene_symbol": "IFNW1",
  "term_id": "GO:0005125",
  "gene": "UniProtKB:P05000"
}